host cell cytoplasm [GO:0030430] (cellular component) Also known as: other organism cytoplasm Sources: GOC:mah Definition: The cytoplasm of a host cell. Relationships: is a type of host intracellular part [GO:0033646]